positive regulation of endothelial cell apoptotic process [GO:2000353] (biological process) Relationships: is a type of positive regulation of apoptotic process [GO:0043065]; is a type of regulation of endothelial cell apoptotic process [GO:2000351]; positively regulates endothelial cell apoptotic process [GO:0072577] Also known as: positive regulation of apoptosis of endothelial cells, positive regulation of endothelial cell programmed cell death by apoptosis, positive regulation of killing of endothelial cells, positive regulation of programmed cell death of endothelial cells by apoptosis, positive regulation of programmed cell death, endothelial cells, positive regulation of endothelial cell apoptosis Definition: Any process that activates or increases the frequency, rate or extent of endothelial cell apoptotic process. Sources: GOC:BHF, GOC:mah, GOC:mtg_apoptosis